negative regulation of postsynaptic density organization [GO:1905875] (biological process) Definition: Any process that stops, prevents or reduces the frequency, rate or extent of postsynaptic density organization. Subtypes: negative regulation of postsynaptic density assembly [GO:0160037] Relationships: is a type of GO:0010639; is a type of regulation of postsynaptic density organization [GO:1905874]; RO_0002212 postsynaptic density organization [GO:0097106] References: PMID:21887379 Sources: GOC:TermGenie, GO_REF:0000058 Also known as: down regulation of PSD organization, down regulation of post synaptic density organization, down regulation of post-synaptic density organization, down regulation of postsynaptic density organisation, down regulation of postsynaptic density organization, down-regulation of PSD organization, down-regulation of post synaptic density organization, down-regulation of post-synaptic density organization, down-regulation of postsynaptic density organisation, down-regulation of postsynaptic density organization, downregulation of PSD organization, downregulation of post synaptic density organization, downregulation of post-synaptic density organization, downregulation of postsynaptic density organisation, downregulation of postsynaptic density organization, negative regulation of PSD organization, negative regulation of post synaptic density organization, negative regulation of post-synaptic density organization, negative regulation of postsynaptic density organisation, inhibition of PSD organization, inhibition of post synaptic density organization, inhibition of post-synaptic density organization, inhibition of postsynaptic density organisation, inhibition of postsynaptic density organization